regulation of short-term neuronal synaptic plasticity [GO:0048172] (biological process) Definition: A process that modulates short-term neuronal synaptic plasticity, the ability of neuronal synapses to change in the short-term as circumstances require. Short-term neuronal synaptic plasticity generally involves increasing or decreasing synaptic sensitivity. References: PMID:11891290 Sources: GOC:jid Note: Note that the syntax of the definition of this term is different from the usual regulation syntax because it describes regulation of a trait rather than regulation of a process. Relationships: is a type of regulation of neuronal synaptic plasticity [GO:0048168] Subtypes: GO:0048173, negative regulation of short-term neuronal synaptic plasticity [GO:0048174]